platelet activating factor production involved in inflammatory response [GO:0002391] (biological process) Definition: The synthesis or release of platelet activating factor following a stimulus as part of an inflammatory response, resulting in an increase in its intracellular or extracellular levels. Sources: GOC:add, ISBN:0781735149 Also known as: platelet activating factor production involved in acute inflammatory response, platelet activating factor secretion, platelet activating factor secretion involved in acute inflammatory response, platelet activating factor secretion involved in inflammatory response, platelet activating factor production Relationships: is a type of production of molecular mediator involved in inflammatory response [GO:0002532]; has part GO:0006663